{
  "gene_symbol": "SPDYE3",
  "term_id": "UNKNOWN:0003",
  "term_label": "Unknown cellular component",
  "gene": "UniProtKB:A6NKU9",
  "gene_name": "Speedy protein E3"
}